{
  "gene_symbol": "NCF1B",
  "term_id": "GO:0016176",
  "term_label": "superoxide-generating NADPH oxidase activator activity",
  "gene": "UniProtKB:A6NI72",
  "gene_name": "Putative neutrophil cytosol factor 1B"
}